{
  "term_label": "maturation of SSU-rRNA from tricistronic rRNA transcript (SSU-rRNA, 5.8S rRNA, LSU-rRNA)",
  "gene_symbol": "RPS8",
  "term_id": "GO:0000462",
  "gene_name": "Small ribosomal subunit protein eS8",
  "gene": "UniProtKB:P62241"
}